galactarate O-hydroxycinnamoyltransferase activity [GO:0047169] (molecular function) Definition: Catalysis of the reaction: feruloyl-CoA + galactarate = 2-(E)-O-feruloyl-D-galactarate + CoA. Relationships: is a type of O-hydroxycinnamoyltransferase activity [GO:0050737] Also known as: feruloyl-CoA:galactarate O-(hydroxycinnamoyl)transferase activity, galacturate hydroxycinnamoyltransferase activity Sources: EC:2.3.1.130, RHEA:12997